{
  "gene": "UniProtKB:Q92615",
  "gene_symbol": "LARP4B",
  "gene_name": "La-related protein 4B",
  "term_label": "cytosol",
  "term_id": "GO:0005829"
}